{
  "gene_symbol": "VDR",
  "term_id": "GO:0000122",
  "gene_name": "Vitamin D3 receptor",
  "gene": "UniProtKB:P11473",
  "term_label": "negative regulation of transcription by RNA polymerase II"
}